{
  "gene_symbol": "STAT2",
  "term_label": "defense response",
  "gene_name": "Signal transducer and activator of transcription 2",
  "term_id": "GO:0006952",
  "gene": "UniProtKB:P52630"
}